{
  "gene_symbol": "USP44",
  "term_label": "Unknown molecular function",
  "gene": "UniProtKB:Q9H0E7",
  "term_id": "UNKNOWN:0001",
  "gene_name": "Ubiquitin carboxyl-terminal hydrolase 44"
}